{
  "term_id": "GO:0000981",
  "gene_symbol": "EN1",
  "gene_name": "Homeobox protein engrailed-1",
  "term_label": "DNA-binding transcription factor activity, RNA polymerase II-specific",
  "gene": "UniProtKB:Q05925"
}